2,4-dichlorobenzoate catabolic process [GO:0046298] (BP) Sources: GOC:ai Definition: The chemical reactions and pathways resulting in the breakdown of 2,4-dichlorobenzoate, a chlorinated aromatic compound which is a key intermediate in the aerobic degradation of polychlorinated biphenyls (PCBs). Also known as: 2,4-dichlorobenzoate breakdown, 2,4-dichlorobenzoate catabolism, 2,4-dichlorobenzoate degradation Relationships: is a type of benzene-containing compound metabolic process [GO:0042537]; is a type of monocarboxylic acid catabolic process [GO:0072329]; is a type of organohalogen metabolic process [GO:0090345]